{
  "term_label": "Unknown biological process",
  "gene_name": "Pleckstrin homology domain-containing family A member 5",
  "gene": "UniProtKB:Q9HAU0",
  "gene_symbol": "PLEKHA5",
  "term_id": "UNKNOWN:0002"
}